axonemal doublet microtubule [GO:0097545] (cellular component) References: PMID:5044758, PMID:5664206 Sources: GOC:cilia, GOC:krc, GOC:pr, Wikipedia:Axoneme, https://github.com/geneontology/go-ontology/issues/26128 Also known as: outer doublet, axonemal outer doublet, axoneme outer doublet, DMT, outer-doublet microtubules Definition: A cellular anatomical entity that is part of an axoneme consisting of a doublet microtubule. Relationships: is a type of GO:0110165; is part of axoneme [GO:0005930]; has part GO:0097649; has part GO:0097650